{
  "term_label": "proton transmembrane transport",
  "gene": "UniProtKB:Q96D96",
  "term_id": "GO:1902600",
  "gene_symbol": "HVCN1",
  "gene_name": "Voltage-gated hydrogen channel 1"
}